vesicle coat [GO:0030120] (cellular component) Definition: A membrane coat found on a coated vesicle. Sources: GOC:mah Subtypes: GO:0030125, COPI vesicle coat [GO:0030126], GO:0030127 Relationships: is a type of GO:0030117; is part of coated vesicle membrane [GO:0030662]